{
  "gene_symbol": "SLC26A3",
  "gene_name": "Chloride anion exchanger",
  "term_label": "oxalate transmembrane transporter activity",
  "term_id": "GO:0019531",
  "gene": "UniProtKB:P40879"
}